{
  "gene": "UniProtKB:Q13637",
  "term_label": "mitochondrion",
  "gene_name": "Ras-related protein Rab-32",
  "gene_symbol": "RAB32",
  "term_id": "GO:0005739"
}